xyloglucan-specific endo-beta-1,4-glucanase inhibitor activity [GO:0140594] (molecular function) Relationships: is a type of GO:0004857; negatively regulates GO:0033946 Definition: Stops, prevents or reduces the activity of xyloglucan-specific endo-beta-1,4-glucanase. References: PMID:28082413